N-acetylgalactosamine binding [GO:0046871] (molecular function) Relationships: is a type of carbohydrate derivative binding [GO:0097367] Definition: Binding to N-acetylgalactosamine, 2-acetamido-2-deoxygalactopyranose, the n-acetyl derivative of galactosamine. References: PMID:18384150 Sources: GOC:ai Also known as: N-acetylgalactosamine lectin